{
  "gene": "UniProtKB:Q96CP7",
  "gene_symbol": "TLCD1",
  "gene_name": "TLC domain-containing protein 1",
  "term_id": "GO:0005886",
  "term_label": "plasma membrane"
}